{
  "gene_symbol": "WASH3P",
  "gene_name": "Putative WAS protein family homolog 3",
  "gene": "UniProtKB:C4AMC7",
  "term_label": "early endosome",
  "term_id": "GO:0005769"
}